mitocytosis [GO:0160040] (biological process) Definition: A migrasome-mediated selective removal of damaged mitochondria process that maintains mitochondrion homeostasis in migrating cells. Relationships: is a type of mitochondrion distribution [GO:0048311]; is a type of GO:0051654; is_a GO:0140495 References: PMID:34108688